{
  "gene_name": "Charged multivesicular body protein 2a",
  "term_id": "GO:0005771",
  "gene_symbol": "CHMP2A",
  "term_label": "multivesicular body",
  "gene": "UniProtKB:O43633"
}